{
  "gene_name": "Olfactory receptor 3A3",
  "term_id": "GO:0004984",
  "gene_symbol": "OR3A3",
  "gene": "UniProtKB:P47888",
  "term_label": "olfactory receptor activity"
}